regulation of hormone metabolic process [GO:0032350] (biological process) Sources: GOC:mah Definition: Any process that modulates the frequency, rate or extent of the chemical reactions and pathways involving any hormone. Subtypes: regulation of ecdysteroid metabolic process [GO:0007553], regulation of glucocorticoid metabolic process [GO:0031943], GO:0032344, GO:0032351, GO:0032352, regulation of juvenile hormone catabolic process [GO:0045952], regulation of hormone biosynthetic process [GO:0046885], regulation of peptide hormone processing [GO:0060568], regulation of auxin metabolic process [GO:0090354], regulation of retinoic acid biosynthetic process [GO:1900052], regulation of thyroid hormone generation [GO:2000609] Relationships: is a type of regulation of hormone levels [GO:0010817]; is a type of regulation of metabolic process [GO:0019222]; RO_0002211 hormone metabolic process [GO:0042445] Also known as: regulation of hormone metabolism